{
  "gene_name": "Interleukin-1 receptor-associated kinase 3",
  "gene": "UniProtKB:Q9Y616",
  "term_label": "interleukin-1-mediated signaling pathway",
  "gene_symbol": "IRAK3",
  "term_id": "GO:0070498"
}